{
  "gene": "UniProtKB:Q8NFP9",
  "gene_name": "Neurobeachin",
  "term_label": "cytosol",
  "term_id": "GO:0005829",
  "gene_symbol": "NBEA"
}